apoptotic DNA fragmentation [GO:0006309] (biological process) Note: DNA fragmentation in response to apoptotic signals is achieved through the activity of apoptotic nucleases. In human, these include DNA fragmentation factor (DFF) or caspase-activated DNase (CAD) and endonuclease G (Endo G) (reviewed in PMID:15723341). Caution is needed when apoptotic DNA laddering assays show presence of fragmented DNA. A positive assay may simply reflect the end point of a whole apoptotic process. Unless clear experimental evidence is available to show that a gene product is directly involved in fragmenting DNA, please do not annotate to GO:0006309 'apoptotic DNA fragmentation' and consider annotating instead to a more upstream process such as, e.g., GO:0042981 'regulation of apoptotic process', GO:0006915 'apoptotic process', GO:0097190 'apoptotic signaling pathway'. Also, note that gene products involved in compartmentalization of apoptotic nucleases and in activation or repression of their enzymatic activity should be annotated to the regulation term GO:1902510 'regulation of apoptotic DNA fragmentation' or to one of its children (see PMID:15723341). References: PMID:15723341, PMID:23379520 Sources: GOC:dph, GOC:mah, GOC:mtg_apoptosis, GOC:tb, ISBN:0721639976 Definition: The cleavage of DNA during apoptosis, which usually occurs in two stages: cleavage into fragments of about 50 kbp followed by cleavage between nucleosomes to yield 200 bp fragments. Also known as: DNA fragmentation, chromatinolysis, DNA catabolic process during apoptosis, DNA catabolism during apoptosis, DNA fragmentation involved in apoptotic nuclear change, endonucleolytic DNA catabolic process involved in apoptosis Regulation: regulated by regulation of apoptotic DNA fragmentation [GO:1902510]; negatively regulated by GO:1902511; RO_0002213 by positive regulation of apoptotic DNA fragmentation [GO:1902512] Relationships: is a type of GO:0006308; is part of apoptotic nuclear changes [GO:0030262]